N-methylalanine dehydrogenase activity [GO:0050132] (molecular function) Definition: Catalysis of the reaction: N-methyl-L-alanine + H2O + NADP+ = H+ + methylammonium + NADPH + pyruvate. Also known as: N-methyl-L-alanine:NADP+ oxidoreductase (demethylating, deaminating) Sources: EC:1.4.1.17, RHEA:21768 Relationships: is a type of oxidoreductase activity, acting on the CH-NH2 group of donors, NAD or NADP as acceptor [GO:0016639]